negative regulation of interleukin-37 production [GO:0150138] (biological process) Relationships: is a type of GO:0001818; is a type of regulation of interleukin-37 production [GO:0150136]; negatively regulates interleukin-37 production [GO:0150137] Also known as: negative regulation of interleukin-37 biosynthetic process References: PMID:30362558 Sources: GOC:aruk Definition: Any process that stops, prevents or reduces the frequency, rate or extent of interleukin-37 production.